{
  "gene_symbol": "TXLNGY",
  "term_id": "UNKNOWN:0003",
  "gene_name": "Putative gamma-taxilin 2",
  "gene": "UniProtKB:Q9BZA5",
  "term_label": "Unknown cellular component"
}